{
  "gene": "UniProtKB:Q3BBV0",
  "term_label": "Unknown biological process",
  "gene_symbol": "NBPF1",
  "gene_name": "Neuroblastoma breakpoint family member 1",
  "term_id": "UNKNOWN:0002"
}